cobalt ion binding [GO:0050897] (molecular function) Sources: GOC:ai Relationships: is a type of transition metal ion binding [GO:0046914] Also known as: Co ion binding, cobalt binding Definition: Binding to a cobalt ion (Co2+).